chromosome, telomeric repeat region [GO:0140445] (cellular component) Relationships: is a type of GO:0000781 Definition: A complex of DNA and protein that seals the end of a chromosome. The telomeric repeat DNA consists of simple tandemly repeated sequences specific for each species. Typically one strand is G-rich and the other C-rich. The G-rich strand forms a 3'-terminal overhang, the length of which varies with species. The single strand overhang is bound by a variety of proteins, including telomere capping proteins that bind to the single-stranded DNA and seal the telomeric loop. References: PMID:11352055, PMID:30208292